{
  "gene_name": "T cell receptor beta variable 12-3",
  "gene_symbol": "TRBV12-3",
  "term_label": "cell surface receptor signaling pathway",
  "term_id": "GO:0007166",
  "gene": "UniProtKB:P01733"
}